{
  "gene_symbol": "PTPN1",
  "term_id": "GO:0005769",
  "gene_name": "Tyrosine-protein phosphatase non-receptor type 1",
  "term_label": "early endosome",
  "gene": "UniProtKB:P18031"
}